negative regulation of pro-T cell differentiation [GO:2000175] (biological process) Definition: Any process that stops, prevents, or reduces the frequency, rate or extent of pro-T cell differentiation. Sources: GOC:BHF Also known as: negative regulation of pro-T lymphocyte differentiation Relationships: is_a negative regulation of T cell differentiation [GO:0045581]; is a type of negative regulation of lymphoid progenitor cell differentiation [GO:1905457]; is a type of regulation of pro-T cell differentiation [GO:2000174]; negatively regulates pro-T cell differentiation [GO:0002572]